artery smooth muscle contraction [GO:0014824] (biological process) Subtypes: arteriole smooth muscle contraction [GO:0014830] Sources: GOC:mtg_muscle, MA:0000708, MSH:D001158 Relationships: is a type of tonic smooth muscle contraction [GO:0014820]; is a type of vascular associated smooth muscle contraction [GO:0014829] Regulation: regulated by regulation of artery smooth muscle contraction [GO:1905654]; negatively regulated by GO:1905655; RO_0002213 by positive regulation of artery smooth muscle contraction [GO:1905656] Definition: A process in which force is generated within smooth muscle tissue, resulting in a change in muscle geometry. This process occurs in the artery. Force generation involves a chemo-mechanical energy conversion step that is carried out by the actin/myosin complex activity, which generates force through ATP hydrolysis. The artery is a vessel carrying blood away from the heart.